{
  "term_label": "RNA polymerase II cis-regulatory region sequence-specific DNA binding",
  "term_id": "GO:0000978",
  "gene_name": "Aryl hydrocarbon receptor nuclear translocator 2",
  "gene_symbol": "ARNT2",
  "gene": "UniProtKB:Q9HBZ2"
}